2,4-dichlorobenzoyl-CoA reductase activity [GO:0018516] (MF) Sources: RHEA:23076 Also known as: 4-chlorobenzoyl-CoA:NADP+ oxidoreductase (halogenating) Relationships: is a type of oxidoreductase activity, acting on X-H and Y-H to form an X-Y bond [GO:0046992] Definition: Catalysis of the reaction: 4-chlorobenzoyl-CoA + chloride + NADP+ = 2,4-dichlorobenzoyl-CoA + NADPH.